viral capsid, fiber [GO:0098022] (cellular component) Relationships: is a type of GO:0098021 Definition: A type of capsid decoration composed of fiber structures. Subtypes: icosahedral viral capsid, collar fiber [GO:0098032], icosahedral viral capsid, neck fiber [GO:0098033] Also known as: head/capsid fiber Sources: GOC:bm